{
  "term_id": "UNKNOWN:0001",
  "gene_name": "Uncharacterized protein C11orf24",
  "gene": "UniProtKB:Q96F05",
  "term_label": "Unknown molecular function",
  "gene_symbol": "C11orf24"
}